{
  "term_id": "GO:0038023",
  "term_label": "signaling receptor activity",
  "gene_name": "Integrin alpha-E",
  "gene": "UniProtKB:P38570",
  "gene_symbol": "ITGAE"
}